{
  "gene": "UniProtKB:Q13322",
  "gene_name": "Growth factor receptor-bound protein 10",
  "term_label": "negative regulation of insulin receptor signaling pathway",
  "term_id": "GO:0046627",
  "gene_symbol": "GRB10"
}